{
  "gene_symbol": "TUBB",
  "gene_name": "Tubulin beta chain",
  "term_label": "mitotic cell cycle",
  "term_id": "GO:0000278",
  "gene": "UniProtKB:P07437"
}